{
  "gene_name": "Checkpoint protein HUS1B",
  "term_label": "checkpoint clamp complex",
  "term_id": "GO:0030896",
  "gene": "UniProtKB:Q8NHY5",
  "gene_symbol": "HUS1B"
}